{
  "term_label": "positive regulation of transcription by RNA polymerase II",
  "term_id": "GO:0045944",
  "gene": "UniProtKB:Q9BYU1",
  "gene_name": "Pre-B-cell leukemia transcription factor 4",
  "gene_symbol": "PBX4"
}